{
  "term_id": "GO:0008028",
  "gene": "UniProtKB:O15374",
  "gene_name": "Monocarboxylate transporter 5",
  "gene_symbol": "SLC16A4",
  "term_label": "monocarboxylic acid transmembrane transporter activity"
}